gibberellin catabolic process [GO:0045487] (biological process) Also known as: gibberellin catabolism, gibberellic acid breakdown, gibberellic acid catabolic process, gibberellic acid catabolism, gibberellic acid degradation Relationships: is a type of GO:0009685; is a type of diterpenoid catabolic process [GO:0016103]; is a type of carboxylic acid catabolic process [GO:0046395] Definition: The chemical reactions and pathways resulting in the breakdown of gibberellin. Gibberellins are a class of highly modified terpenes that function as plant growth regulators. Sources: GOC:go_curators